lysophosphatidylethanolamine acyltransferase activity [GO:0071618] (molecular function) Relationships: is a type of lysophospholipid acyltransferase activity [GO:0071617] Definition: Catalysis of the transfer of acyl groups from an acyl-CoA to lysophosphatidylethanolamine. Sources: GOC:cjk